{
  "gene_name": "Putative N-acetylated-alpha-linked acidic dipeptidase",
  "term_id": "UNKNOWN:0001",
  "gene_symbol": "FOLH1B",
  "term_label": "Unknown molecular function",
  "gene": "UniProtKB:Q9HBA9"
}